gluconate dehydratase activity [GO:0047929] (molecular function) Definition: Catalysis of the reaction: D-gluconate = 2-dehydro-3-deoxy-D-gluconate + H2O. Relationships: is a type of hydro-lyase activity [GO:0016836] Sources: EC:4.2.1.39, RHEA:21612 Also known as: D-gluconate dehydratase activity, D-gluconate hydro-lyase (2-dehydro-3-deoxy-D-gluconate-forming), D-gluconate hydro-lyase activity